IgE immunoglobulin complex [GO:0071742] (cellular component) Note: Note that an IgE immunoglobulin complex has the function of antigen binding if a suitable antigen is available. Definition: A protein complex composed of two identical immunoglobulin heavy chains of the IgE isotype and two identical immunoglobulin light chains, held together by disulfide bonds. An IgE immunoglobulin complex may be embedded in the plasma membrane or present in the extracellular space, in mucosal areas or other tissues, or circulating in the blood or lymph. Sources: GOC:add, ISBN:0781765196 Relationships: is a type of immunoglobulin complex [GO:0019814] Subtypes: GO:0071743, IgE B cell receptor complex [GO:0071744]